{
  "gene_name": "Leiomodin-2",
  "gene_symbol": "LMOD2",
  "term_id": "GO:0005865",
  "gene": "UniProtKB:Q6P5Q4",
  "term_label": "striated muscle thin filament"
}